methylenetetrahydrofolate dehydrogenase (NAD+) activity [GO:0004487] (molecular function) Definition: Catalysis of the reaction: 5,10-methylenetetrahydrofolate + NAD+ = 5,10-methenyltetrahydrofolate + NADH. Sources: RHEA:22892 Also known as: 5,10-methylenetetrahydrofolate dehydrogenase activity, 5,10-methylenetetrahydrofolate:NAD+ oxidoreductase Relationships: is a type of oxidoreductase activity, acting on the CH-NH group of donors, NAD or NADP as acceptor [GO:0016646]